oxidoreductase activity, acting on the aldehyde or oxo group of donors, iron-sulfur protein as acceptor [GO:0016625] (molecular function) Definition: Catalysis of an oxidation-reduction (redox) reaction in which an aldehyde or ketone (oxo) group acts as a hydrogen or electron donor and reduces an iron-sulfur protein. Also known as: oxidoreductase activity, acting on the aldehyde or oxo group of donors, iron-sulphur protein as acceptor Relationships: is a type of oxidoreductase activity, acting on the aldehyde or oxo group of donors [GO:0016903] Subtypes: pyruvate synthase activity [GO:0019164], aldehyde ferredoxin oxidoreductase activity [GO:0033726], glyceraldehyde-3-phosphate dehydrogenase (ferredoxin) activity [GO:0043797], indolepyruvate ferredoxin oxidoreductase activity [GO:0043805], 3-methyl-2-oxobutanoate dehydrogenase (ferredoxin) activity [GO:0043807], pyruvate-flavodoxin oxidoreductase activity [GO:0043873], anaerobic carbon-monoxide dehydrogenase activity [GO:0043885], 2-oxoglutarate synthase activity [GO:0047553] Sources: GOC:jl